{
  "gene_symbol": "LATS2",
  "term_id": "GO:0004674",
  "term_label": "protein serine/threonine kinase activity",
  "gene_name": "Serine_threonine-protein kinase LATS2",
  "gene": "UniProtKB:Q9NRM7"
}